symbiont-mediated suppression of host JAK-STAT cascade via inhibition of STAT1 activity [GO:0039563] (biological process) References: PMID:32699158 Relationships: is a type of symbiont-mediated suppression of host JAK-STAT cascade via inhibition of STAT activity [GO:0039562] Definition: A process in which a symbiont interferes with, inhibits or disrupt a JAK-STAT signal cascade in the host organism by reducing the activity of host STAT1 (signal transducer and activator of transcription 1). Note: This term is for annotation of symbiont proteins that counteract the host innate immune response. Also known as: disruption by virus of host JAK-STAT cascade via inhibition of STAT1 activity, inhibition by virus of host STAT1 activity, inhibition of host STAT1 by virus, suppression by virus of host JAK-STAT cascade via inhibition of STAT1 activity, suppression by virus of host STAT1 activity